germinal center B cell differentiation [GO:0002314] (biological process) Note: Note that immunologists typically use the word 'development' to refer to cells of B or T cell lineages undergoing the process that GO describes as 'cell differentiation'. Definition: The process in which a B cell in the spleen acquires the specialized features of a germinal center B cell. Germinal center B cells are rapidly cycling B cells which have downregulated IgD expression and exhibit high levels of binding by peanut agglutinin (PNA). Sources: GOC:jal, ISBN:0781735149 Relationships: is a type of mature B cell differentiation involved in immune response [GO:0002313] Also known as: germinal center B lymphocyte differentiation, germinal center B-cell differentiation, germinal center B-lymphocyte differentiation, germinal center B cell development